{
  "term_label": "microtubule-based movement",
  "gene_name": "Kinesin light chain 1",
  "gene": "UniProtKB:Q07866",
  "gene_symbol": "KLC1",
  "term_id": "GO:0007018"
}